{
  "term_label": "regulation of transcription by RNA polymerase II",
  "gene_symbol": "ZSCAN5A",
  "gene_name": "Zinc finger and SCAN domain-containing protein 5A",
  "gene": "UniProtKB:Q9BUG6",
  "term_id": "GO:0006357"
}